{
  "term_id": "UNKNOWN:0001",
  "gene_symbol": "ZSWIM8",
  "term_label": "Unknown molecular function",
  "gene_name": "Zinc finger SWIM domain-containing protein 8",
  "gene": "UniProtKB:A7E2V4"
}